{
  "gene_name": "Fibronectin type III domain-containing protein 11",
  "gene": "UniProtKB:Q9BVV2",
  "gene_symbol": "FNDC11",
  "term_label": "Unknown cellular component",
  "term_id": "UNKNOWN:0003"
}